{
  "gene_name": "Anaphase-promoting complex subunit 11",
  "gene_symbol": "ANAPC11",
  "term_id": "GO:0005680",
  "gene": "UniProtKB:Q9NYG5",
  "term_label": "anaphase-promoting complex"
}